pantothenase activity [GO:0004593] (molecular function) Definition: Catalysis of the reaction: (R)-pantothenate + H2O = (R)-pantoate + beta-alanine. Relationships: is a type of hydrolase activity, acting on carbon-nitrogen (but not peptide) bonds, in linear amides [GO:0016811] Sources: EC:3.5.1.22, RHEA:12448 Also known as: (R)-pantothenate amidohydrolase activity, pantothenate amidohydrolase activity, pantothenate hydrolase activity